{
  "term_id": "GO:0007274",
  "gene": "UniProtKB:P02708",
  "gene_name": "Acetylcholine receptor subunit alpha",
  "gene_symbol": "CHRNA1",
  "term_label": "neuromuscular synaptic transmission"
}